regulation of T cell differentiation in thymus [GO:0033081] (biological process) Subtypes: negative regulation of T cell differentiation in thymus [GO:0033085], positive regulation of T cell differentiation in thymus [GO:0033089], regulation of positive thymic T cell selection [GO:1902232] Sources: GOC:add, GOC:mah Definition: Any process that modulates the frequency, rate or extent of T cell differentiation in the thymus. Also known as: regulation of thymic T cell differentiation, regulation of thymocyte cell differentiation, regulation of thymocyte differentiation, regulation of T cell development in thymus Note: Note that immunologists typically use the word 'development' to refer to cells of B or T cell lineages undergoing the process that GO describes as 'cell differentiation'. Relationships: is a type of GO:0045580; regulates GO:0033077